{
  "gene_name": "Peroxisomal succinyl-coenzyme A thioesterase",
  "gene": "UniProtKB:Q8N9L9",
  "gene_symbol": "ACOT4",
  "term_id": "GO:0006631",
  "term_label": "fatty acid metabolic process"
}